{
  "gene_name": "Calcineurin subunit B type 1",
  "gene": "UniProtKB:P63098",
  "term_id": "GO:0019902",
  "gene_symbol": "PPP3R1",
  "term_label": "phosphatase binding"
}